type 2 proteinase activated receptor binding [GO:0031873] (molecular function) Also known as: type 2 proteinase activated receptor ligand Definition: Binding to a type 2 proteinase activated receptor. Sources: GOC:mah, GOC:nln Relationships: is a type of proteinase activated receptor binding [GO:0031871]